{
  "gene": "UniProtKB:Q5JQF7",
  "term_label": "Unknown molecular function",
  "gene_symbol": "LINC01556",
  "gene_name": "Putative uncharacterized protein encoded by LINC01556",
  "term_id": "UNKNOWN:0001"
}